{
  "gene_name": "Ret finger protein-like 1",
  "gene": "UniProtKB:O75677",
  "gene_symbol": "RFPL1",
  "term_label": "innate immune response",
  "term_id": "GO:0045087"
}